{
  "gene_name": "Membrane-spanning 4-domains subfamily A member 15",
  "gene_symbol": "MS4A15",
  "term_label": "Unknown molecular function",
  "gene": "UniProtKB:Q8N5U1",
  "term_id": "UNKNOWN:0001"
}